{
  "gene_symbol": "CALR3",
  "gene_name": "Calreticulin-3",
  "gene": "UniProtKB:Q96L12",
  "term_id": "GO:0006457",
  "term_label": "protein folding"
}